{
  "term_label": "pre-mRNA 3'-splice site binding",
  "gene": "UniProtKB:Q8WU68",
  "gene_name": "Splicing factor U2AF 26 kDa subunit",
  "gene_symbol": "U2AF1L4",
  "term_id": "GO:0030628"
}